{
  "gene_name": "Chymase",
  "gene": "UniProtKB:P23946",
  "term_label": "extracellular space",
  "gene_symbol": "CMA1",
  "term_id": "GO:0005615"
}